{
  "gene_name": "Protein MMS22-like",
  "gene": "UniProtKB:Q6ZRQ5",
  "gene_symbol": "MMS22L",
  "term_id": "GO:0000724",
  "term_label": "double-strand break repair via homologous recombination"
}